{
  "gene_name": "Chemokine-like protein TAFA-1",
  "gene_symbol": "TAFA1",
  "gene": "UniProtKB:Q7Z5A9",
  "term_id": "GO:0005615",
  "term_label": "extracellular space"
}